{
  "term_id": "UNKNOWN:0002",
  "term_label": "Unknown biological process",
  "gene_symbol": "GPALPP1",
  "gene": "UniProtKB:Q8IXQ4",
  "gene_name": "GPALPP motifs-containing protein 1"
}